{
  "gene": "UniProtKB:Q9C0B6",
  "term_id": "GO:0071300",
  "gene_symbol": "BRINP2",
  "term_label": "cellular response to retinoic acid",
  "gene_name": "BMP_retinoic acid-inducible neural-specific protein 2"
}